mitotic cell cycle process [GO:1903047] (BP) Definition: A process that is part of the mitotic cell cycle. Sources: GOC:TermGenie, GOC:mtg_cell_cycle, GO_REF:0000060 Relationships: is_a GO:0022402; is part of mitotic cell cycle [GO:0000278] Subtypes: mitotic spindle elongation [GO:0000022], GO:0000070, initial mitotic spindle pole body separation [GO:0000073], mitotic cytokinesis [GO:0000281], GO:0000282, mitotic chromosome condensation [GO:0007076], mitotic nuclear membrane disassembly [GO:0007077], lamin depolymerization [GO:0007078], mitotic chromosome movement towards spindle pole [GO:0007079], mitotic metaphase chromosome alignment [GO:0007080], GO:0007087, GO:0007093, mitotic centrosome separation [GO:0007100], GO:0009833, GO:0009920, cellular bud neck septin ring organization [GO:0032186], establishment of mitotic sister chromatid cohesion [GO:0034087], mitotic cell cycle phase transition [GO:0044772], mitotic spindle midzone assembly [GO:0051256], GO:0051306, GO:0051315, karyomere assembly [GO:0061471], karyomere membrane fusion [GO:0061472], centromere clustering at the mitotic interphase nuclear envelope [GO:0072766], microtubule plus-end directed mitotic chromosome migration [GO:0099606], mitotic nuclear membrane organization [GO:0101024], GO:0101026, mitotic nuclear division [GO:0140014], repair of mitotic kinetochore microtubule attachment defect [GO:0140273], mitotic nuclear envelope segregation [GO:0160052], mitotic actomyosin contractile ring maturation [GO:1902406], GO:1902410, microtubule cytoskeleton organization involved in mitosis [GO:1902850], mitotic DNA replication [GO:1902969], mitotic DNA replication initiation [GO:1902975], mitotic DNA replication preinitiation complex assembly [GO:1902977], mitotic DNA replication termination [GO:1902979], DNA strand elongation involved in mitotic DNA replication [GO:1902983], mitotic pre-replicative complex assembly [GO:1902985], GO:1902990, mitotic spindle pole body duplication [GO:1903087], GO:1903461, GO:1903469, mitotic actomyosin contractile ring assembly actin filament organization [GO:1903479], DNA synthesis involved in mitotic DNA replication [GO:1904860], mitotic DNA replication maintenance of fidelity [GO:1990505], GO:1990608, mitotic sister chromatid arm separation [GO:1990891]